morphogenesis of embryonic epithelium [GO:0016331] (biological process) Sources: GOC:jl Relationships: is a type of GO:0002009; is_a embryonic morphogenesis [GO:0048598] Definition: The process in which the anatomical structures of embryonic epithelia are generated and organized. Subtypes: neural plate morphogenesis [GO:0001839], GO:0001842, optic cup morphogenesis involved in camera-type eye development [GO:0002072], anterior midgut invagination [GO:0007375], GO:0007391, GO:0021506, posterior neuropore closure [GO:0021507], progression of neural tube closure [GO:0021994], GO:0021995, GO:0048615, GO:0060431, GO:0060513, mammary gland bud formation [GO:0060615], mammary gland cord formation [GO:0060616]